L-ascorbic acid transmembrane transport [GO:0015882] (biological process) Also known as: L-ascorbate transport, vitamin C transport, L-ascorbic acid transport Relationships: is a type of monosaccharide transmembrane transport [GO:0015749]; is a type of GO:0035461; is a type of GO:1905039 Sources: GOC:ai Definition: The process in which L-ascorbic acid is transported across a lipid bilayer, from one side of a membrane to the other. L-ascorbate, (2R)-2-[(1S)-1,2-dihydroxyethyl]-4-hydroxy-5-oxo-2,5-dihydrofuran-3-olate, is vitamin C and has co-factor and anti-oxidant activities in many species.